{
  "term_id": "GO:0005634",
  "gene_name": "RecQ-like DNA helicase BLM",
  "term_label": "nucleus",
  "gene": "UniProtKB:P54132",
  "gene_symbol": "BLM"
}